{
  "gene": "UniProtKB:O75608",
  "gene_symbol": "LYPLA1",
  "term_label": "palmitoyl-(protein) hydrolase activity",
  "term_id": "GO:0008474",
  "gene_name": "Acyl-protein thioesterase 1"
}